{
  "gene": "UniProtKB:Q53H76",
  "term_label": "phospholipase A1 activity",
  "term_id": "GO:0008970",
  "gene_name": "Phospholipase A1 member A",
  "gene_symbol": "PLA1A"
}